{
  "gene_symbol": "PRPF18",
  "term_label": "U5 snRNP",
  "gene_name": "Pre-mRNA-splicing factor 18",
  "gene": "UniProtKB:Q99633",
  "term_id": "GO:0005682"
}